{
  "gene_name": "Transcription activator BRG1",
  "term_id": "GO:0003677",
  "gene_symbol": "SMARCA4",
  "term_label": "DNA binding",
  "gene": "UniProtKB:P51532"
}